{
  "gene": "UniProtKB:Q8NG68",
  "term_id": "GO:0004835",
  "gene_name": "Tubulin--tyrosine ligase",
  "gene_symbol": "TTL",
  "term_label": "tubulin-tyrosine ligase activity"
}